{
  "gene": "UniProtKB:P06702",
  "gene_symbol": "S100A9",
  "term_id": "GO:0048306",
  "term_label": "calcium-dependent protein binding",
  "gene_name": "Protein S100-A9"
}